{
  "gene_symbol": "OR4C15",
  "gene_name": "Olfactory receptor 4C15",
  "term_label": "plasma membrane",
  "term_id": "GO:0005886",
  "gene": "UniProtKB:Q8NGM1"
}